{
  "gene": "UniProtKB:P47895",
  "term_id": "GO:0004029",
  "term_label": "aldehyde dehydrogenase (NAD+) activity",
  "gene_symbol": "ALDH1A3",
  "gene_name": "Retinaldehyde dehydrogenase 3"
}